{
  "term_label": "calcium-mediated signaling",
  "gene_name": "Kinase suppressor of Ras 2",
  "gene": "UniProtKB:Q6VAB6",
  "term_id": "GO:0019722",
  "gene_symbol": "KSR2"
}